{
  "gene_name": "Biogenesis of lysosome-related organelles complex 1 subunit 1",
  "gene": "UniProtKB:P78537",
  "term_label": "endosomal transport",
  "term_id": "GO:0016197",
  "gene_symbol": "BLOC1S1"
}